{
  "gene_symbol": "TIMP3",
  "term_id": "GO:0009725",
  "gene_name": "Metalloproteinase inhibitor 3",
  "term_label": "response to hormone",
  "gene": "UniProtKB:P35625"
}